{
  "term_id": "GO:0005886",
  "gene_name": "Protein ELFN1",
  "term_label": "plasma membrane",
  "gene": "UniProtKB:P0C7U0",
  "gene_symbol": "ELFN1"
}